{
  "term_id": "GO:0005834",
  "gene_name": "Guanine nucleotide-binding protein subunit alpha-14",
  "term_label": "heterotrimeric G-protein complex",
  "gene_symbol": "GNA14",
  "gene": "UniProtKB:O95837"
}